retinal cone cell fate commitment [GO:0046551] (BP) Relationships: is a type of camera-type eye photoreceptor cell fate commitment [GO:0060220]; is part of GO:0042670 Regulation: regulated by regulation of retinal cone cell fate commitment [GO:0060222]; negatively regulated by GO:0060226 Definition: The process in which the developmental fate of a cell becomes restricted such that it will develop into a retinal cone cell. A retinal cone cell is one of the two photoreceptor subtypes in a camera-type eye. References: PMID:3076112, PMID:3937883 Sources: GOC:mtg_sensu